{
  "term_label": "Unknown molecular function",
  "gene_name": "Rho guanine nucleotide exchange factor 39",
  "term_id": "UNKNOWN:0001",
  "gene_symbol": "ARHGEF39",
  "gene": "UniProtKB:Q8N4T4"
}